type II site-specific deoxyribonuclease activity [GO:0009036] (molecular function) References: PMID:12654995 Sources: EC:3.1.21.4 Also known as: type II restriction enzyme activity Definition: Catalysis of the endonucleolytic cleavage of DNA to give specific double-stranded fragments with terminal 5'-phosphates and 3' hydroxyls. Cleavage is dependent on the presence in the DNA of a specific recognition site; cleavage occurs at or very near this recognition site. Relationships: is a type of restriction endodeoxyribonuclease activity [GO:0015666]; is a type of DNA endonuclease activity, producing 5'-phosphomonoesters [GO:0016888]